{
  "gene_name": "Y+L amino acid transporter 1",
  "gene_symbol": "SLC7A7",
  "term_label": "Unknown cellular component",
  "term_id": "UNKNOWN:0003",
  "gene": "UniProtKB:Q9UM01"
}